{
  "gene_symbol": "RBP3",
  "term_id": "GO:0019841",
  "term_label": "retinol binding",
  "gene": "UniProtKB:P10745",
  "gene_name": "Retinol-binding protein 3"
}